{
  "gene": "UniProtKB:Q9H3R0",
  "term_label": "chromatin",
  "gene_name": "Lysine-specific demethylase 4C",
  "gene_symbol": "KDM4C",
  "term_id": "GO:0000785"
}